{
  "term_label": "olfactory receptor activity",
  "gene_name": "Olfactory receptor 5AN1",
  "gene": "UniProtKB:Q8NGI8",
  "term_id": "GO:0004984",
  "gene_symbol": "OR5AN1"
}